plastid ribosome [GO:0009547] (cellular component) Definition: A ribosome contained within a plastid. Relationships: is a type of organellar ribosome [GO:0000313]; is part of plastid stroma [GO:0009532] Sources: GOC:tair_curators Subtypes: chloroplast ribosome [GO:0043253]